{
  "gene": "UniProtKB:Q9UPR6",
  "gene_symbol": "ZFR2",
  "term_label": "single-stranded RNA binding",
  "term_id": "GO:0003727",
  "gene_name": "Zinc finger RNA-binding protein 2"
}